pyruvate-flavodoxin oxidoreductase activity [GO:0043873] (molecular function) Definition: Catalysis of the reaction: pyruvate + CoA + oxidized flavodoxin = acetyl-CoA + CO2 + reduced flavodoxin. References: PMID:6352705 Relationships: is a type of oxidoreductase activity, acting on the aldehyde or oxo group of donors, iron-sulfur protein as acceptor [GO:0016625] Also known as: pyruvate:flavodoxin oxidoreductase activity, NifJ